{
  "term_label": "immunoglobulin complex",
  "gene": "UniProtKB:A0A0C4DH24",
  "term_id": "GO:0019814",
  "gene_name": "Immunoglobulin kappa variable 6-21",
  "gene_symbol": "IGKV6-21"
}